{
  "gene_name": "Protein ABHD1",
  "term_label": "acetylesterase activity",
  "term_id": "GO:0008126",
  "gene_symbol": "ABHD1",
  "gene": "UniProtKB:Q96SE0"
}